ferulate 5-hydroxylase activity [GO:0046424] (molecular function) Relationships: is a type of monooxygenase activity [GO:0004497]; is_a GO:0016651 Definition: Catalysis of the reaction: ferulic acid + NADPH + H+ + O2 = 5-hydroxyferulic acid + H2O + NADP+. References: PMID:8692910, PMID:9880351